{
  "gene_symbol": "JUP",
  "term_id": "GO:0016922",
  "gene_name": "Junction plakoglobin",
  "term_label": "nuclear receptor binding",
  "gene": "UniProtKB:P14923"
}